{
  "term_id": "GO:0033038",
  "term_label": "bitter taste receptor activity",
  "gene_symbol": "TAS2R7",
  "gene": "UniProtKB:Q9NYW3",
  "gene_name": "Taste receptor type 2 member 7"
}